{
  "gene_name": "Ufm1-specific protease 2",
  "gene_symbol": "UFSP2",
  "term_label": "nucleus",
  "gene": "UniProtKB:Q9NUQ7",
  "term_id": "GO:0005634"
}